{
  "gene": "UniProtKB:Q8IW36",
  "gene_name": "Zinc finger protein 695",
  "gene_symbol": "ZNF695",
  "term_id": "GO:0000978",
  "term_label": "RNA polymerase II cis-regulatory region sequence-specific DNA binding"
}